{
  "gene_symbol": "TRPC4",
  "term_id": "GO:0005886",
  "gene_name": "Short transient receptor potential channel 4",
  "gene": "UniProtKB:Q9UBN4",
  "term_label": "plasma membrane"
}